glucosinolate transmembrane transporter activity [GO:0141165] (molecular function) Definition: Enables the transfer of a glucosinolate across a membrane. Relationships: is a type of carbohydrate derivative transmembrane transporter activity [GO:1901505]; is a type of sulfur compound transmembrane transporter activity [GO:1901682] References: PMID:37076627 Subtypes: GO:0090448